riboflavin reductase [NAD(P)H] activity [GO:0052875] (molecular function) Also known as: riboflavin reductase (NADH) activity, riboflavin reductase (NADPH) activity, NAD(P)H-FMN reductase activity, NAD(P)H-dependent FMN reductase activity, NAD(P)H2 dehydrogenase (FMN) activity, NAD(P)H2:FMN oxidoreductase activity, NAD(P)H:FMN oxidoreductase activity, NAD(P)H:riboflavin oxidoreductase activity, flavin mononucleotide reductase activity, flavine mononucleotide reductase activity, riboflavin mononucleotide (reduced nicotinamide adenine dinucleotide) reductase activity, riboflavin mononucleotide reductase activity, riboflavine mononucleotide reductase activity Subtypes: GO:0042602 Sources: EC:1.5.1.41 Definition: Catalysis of the reaction: reduced riboflavin + NAD(P)+ = riboflavin + NAD(P)H + 2 H+. This reaction can utilize NADH and NADPH. Relationships: is a type of oxidoreductase activity, acting on the CH-NH group of donors, NAD or NADP as acceptor [GO:0016646]